{
  "term_label": "Unknown molecular function",
  "term_id": "UNKNOWN:0001",
  "gene_symbol": "POLE4",
  "gene": "UniProtKB:Q9NR33",
  "gene_name": "DNA polymerase epsilon subunit 4"
}